{
  "gene_name": "Putative claudin-24",
  "term_label": "plasma membrane",
  "gene": "UniProtKB:A6NM45",
  "term_id": "GO:0005886",
  "gene_symbol": "CLDN24"
}